{
  "gene_name": "Ryanodine receptor 2",
  "gene": "UniProtKB:Q92736",
  "gene_symbol": "RYR2",
  "term_label": "calcium channel complex",
  "term_id": "GO:0034704"
}